{
  "term_label": "regulation of BMP signaling pathway",
  "gene_symbol": "FSTL3",
  "gene": "UniProtKB:O95633",
  "term_id": "GO:0030510",
  "gene_name": "Follistatin-related protein 3"
}